{
  "term_id": "GO:0030020",
  "gene": "UniProtKB:P02458",
  "gene_name": "Collagen alpha-1(II) chain",
  "term_label": "extracellular matrix structural constituent conferring tensile strength",
  "gene_symbol": "COL2A1"
}